phosphatidylinositol 3-kinase/protein kinase B signal transduction [GO:0043491] (biological process) Regulation: regulated by regulation of phosphatidylinositol 3-kinase/protein kinase B signal transduction [GO:0051896]; positively regulated by positive regulation of phosphatidylinositol 3-kinase/protein kinase B signal transduction [GO:0051897]; negatively regulated by negative regulation of phosphatidylinositol 3-kinase/protein kinase B signal transduction [GO:0051898] Definition: An intracellular signaling cassette that starts with phosphatidylinositol 3-kinase (PI3K) activation, production of phosphatidylinositol 3-phosphate (PI3P), activation of PDK1, which recruits and ending with the activation of protein kinase B (PKB, also known as Akt). PI3K is activated by cell surface receptors. Note that PTEN is an inhibitor of the pathway. Relationships: is a type of intracellular signaling cassette [GO:0141124] Also known as: PI3K-PKB/Akt pathway, PI3K/Akt signal transduction, PI3K/PKB signal transduction, phosphatidylinositol 3-kinase signaling/protein kinase B signal transduction, AKT signal transduction, AKT signaling, AKT signaling cascade, AKT signalling cascade, PKB signal transduction, PKB signaling, PKB signaling cascade, PKB signalling cascade, protein kinase B signal transduction, protein kinase B signaling, protein kinase B signaling cascade, protein kinase B signalling cascade References: PMID:20517722, PMID:22952397